{
  "term_id": "UNKNOWN:0002",
  "term_label": "Unknown biological process",
  "gene_name": "Olfactory receptor 9A1",
  "gene": "UniProtKB:Q8NGU1",
  "gene_symbol": "OR9A1P"
}